{
  "term_label": "GABA-A receptor complex",
  "gene_name": "Gamma-aminobutyric acid receptor subunit rho-1",
  "term_id": "GO:1902711",
  "gene_symbol": "GABRR1",
  "gene": "UniProtKB:P24046"
}